{
  "term_id": "UNKNOWN:0003",
  "gene_name": "Endogenous retrovirus group 3 member 1 Env polyprotein",
  "gene": "UniProtKB:Q14264",
  "term_label": "Unknown cellular component",
  "gene_symbol": "ERV3-1"
}